female gonad development [GO:0008585] (biological process) Definition: The process whose specific outcome is the progression of the female gonad over time, from its formation to the mature structure. Sources: GOC:dph, GOC:jid, GOC:tb Also known as: ovarian development, ovary development Relationships: is a type of gonad development [GO:0008406]; is part of GO:0046545 Regulation: regulated by regulation of female gonad development [GO:2000194]; negatively regulated by GO:2000195; positively regulated by GO:2000196